regulation of store-operated calcium entry [GO:2001256] (BP) Subtypes: negative regulation of store-operated calcium entry [GO:0106128], positive regulation of store-operated calcium entry [GO:0106129] Definition: Any process that modulates the frequency, rate or extent of store-operated calcium entry. Relationships: is a type of regulation of calcium ion transport [GO:0051924]; regulates store-operated calcium entry [GO:0002115] Sources: GOC:BHF Also known as: regulation of SOCE, regulation of capacitative calcium entry, regulation of store-operated calcium import, regulation of calcium ion import